{
  "gene_name": "Zinc finger protein 280A",
  "gene": "UniProtKB:P59817",
  "term_id": "GO:0006355",
  "gene_symbol": "ZNF280A",
  "term_label": "regulation of DNA-templated transcription"
}